{
  "gene_name": "Fibroblast growth factor 5",
  "gene": "UniProtKB:P12034",
  "term_id": "GO:0043410",
  "term_label": "positive regulation of MAPK cascade",
  "gene_symbol": "FGF5"
}